{
  "gene_name": "Ribonuclease inhibitor",
  "term_id": "GO:0032311",
  "term_label": "angiogenin-PRI complex",
  "gene": "UniProtKB:P13489",
  "gene_symbol": "RNH1"
}